{
  "gene_symbol": "APOC1",
  "gene_name": "Apolipoprotein C-I",
  "gene": "UniProtKB:P02654",
  "term_label": "fatty acid binding",
  "term_id": "GO:0005504"
}